{
  "term_label": "cytosol",
  "gene_name": "Ubiquitin carboxyl-terminal hydrolase 37",
  "gene": "UniProtKB:Q86T82",
  "term_id": "GO:0005829",
  "gene_symbol": "USP37"
}